{
  "term_id": "GO:0000976",
  "gene_symbol": "ZNF473",
  "gene": "UniProtKB:Q8WTR7",
  "term_label": "transcription cis-regulatory region binding",
  "gene_name": "Zinc finger protein 473"
}